{
  "gene_name": "Enhancer of polycomb homolog 2",
  "term_id": "GO:0006325",
  "term_label": "chromatin organization",
  "gene_symbol": "EPC2",
  "gene": "UniProtKB:Q52LR7"
}